{
  "gene_symbol": "PLBD2",
  "term_label": "Unknown molecular function",
  "term_id": "UNKNOWN:0001",
  "gene": "UniProtKB:Q8NHP8",
  "gene_name": "Putative phospholipase B-like 2"
}